{
  "gene_name": "5'-AMP-activated protein kinase catalytic subunit alpha-1",
  "gene": "UniProtKB:Q13131",
  "term_label": "protein serine/threonine kinase activity",
  "term_id": "GO:0004674",
  "gene_symbol": "PRKAA1"
}